cortical endoplasmic reticulum lumen [GO:0099021] (cellular component) Definition: The volume enclosed by the membranes of the cortical endoplasmic reticulum. Sources: GOC:dos, GOC:vw Relationships: is a type of endoplasmic reticulum lumen [GO:0005788]; is part of cortical endoplasmic reticulum [GO:0032541]